{
  "gene_symbol": "FBL",
  "term_label": "small-subunit processome",
  "gene": "UniProtKB:P22087",
  "gene_name": "rRNA 2'-O-methyltransferase fibrillarin",
  "term_id": "GO:0032040"
}